{
  "term_id": "GO:0005231",
  "term_label": "excitatory extracellular ligand-gated monoatomic ion channel activity",
  "gene_name": "5-hydroxytryptamine receptor 3C",
  "gene": "UniProtKB:Q8WXA8",
  "gene_symbol": "HTR3C"
}